{
  "term_label": "regulation of gene expression",
  "gene": "UniProtKB:P50616",
  "term_id": "GO:0010468",
  "gene_name": "Protein Tob1",
  "gene_symbol": "TOB1"
}